{
  "gene_symbol": "GTSF1L",
  "term_label": "Unknown cellular component",
  "gene_name": "Gametocyte-specific factor 1-like",
  "term_id": "UNKNOWN:0003",
  "gene": "UniProtKB:Q9H1H1"
}